endothelial cell chemotaxis to fibroblast growth factor [GO:0035768] (biological process) Relationships: is a type of cell chemotaxis to fibroblast growth factor [GO:0035766]; is_a endothelial cell chemotaxis [GO:0035767] Sources: CL:0000115, GOC:BHF Definition: The directed movement of an endothelial cell in response to the presence of fibroblast growth factor (FGF). Regulation: regulated by regulation of endothelial cell chemotaxis to fibroblast growth factor [GO:2000544]; negatively regulated by negative regulation of endothelial cell chemotaxis to fibroblast growth factor [GO:2000545]; positively regulated by positive regulation of endothelial cell chemotaxis to fibroblast growth factor [GO:2000546]